negative regulation of shell calcification [GO:1905649] (biological process) Definition: Any process that stops, prevents or reduces the frequency, rate or extent of shell calcification. Also known as: down regulation of shell calcification, down-regulation of shell calcification, downregulation of shell calcification, inhibition of shell calcification References: PMID:14648763 Sources: GOC:TermGenie, GO_REF:0000058 Relationships: is a type of negative regulation of biomineral tissue development [GO:0070168]; is a type of regulation of shell calcification [GO:1905648]; negatively regulates shell calcification [GO:0031215]